response to G1 DNA damage checkpoint signaling [GO:0072432] (biological process) Definition: A process that occurs in response to signals generated as a result of G1/S transition DNA damage checkpoint signaling. Sources: GOC:mtg_cell_cycle Also known as: mitotic cell cycle G1/S transition DNA damage checkpoint effector process, response to mitotic cell cycle G1/S transition DNA damage checkpoint signaling, response to signal involved in mitotic cell cycle G1/S transition DNA damage checkpoint Relationships: is a type of response to mitotic cell cycle checkpoint signaling [GO:0072414]; is a type of response to DNA damage checkpoint signaling [GO:0072423] Regulation: regulated by regulation of response to G1 DNA damage checkpoint signaling [GO:1902155]; positively regulated by GO:1902156